{
  "gene": "UniProtKB:Q9BQI3",
  "term_label": "regulation of translational initiation",
  "gene_symbol": "EIF2AK1",
  "gene_name": "Eukaryotic translation initiation factor 2-alpha kinase 1",
  "term_id": "GO:0006446"
}